{
  "gene_name": "AT-rich interactive domain-containing protein 3B",
  "term_id": "GO:0003677",
  "gene_symbol": "ARID3B",
  "term_label": "DNA binding",
  "gene": "UniProtKB:Q8IVW6"
}